{
  "gene_name": "Coiled-coil domain-containing protein 73",
  "gene": "UniProtKB:Q6ZRK6",
  "term_label": "Unknown molecular function",
  "term_id": "UNKNOWN:0001",
  "gene_symbol": "CCDC73"
}